apical cell fate commitment [GO:0010654] (biological process) Sources: GOC:dph, GOC:tb Definition: The process in which the developmental fate of a cell becomes restricted such that it will develop into an apical cell. The apical cell is the upper cell formed after the first division of the zygote. Relationships: is a type of GO:0003006; is a type of cell fate commitment [GO:0045165]; BFO_0000050 embryo development ending in seed dormancy [GO:0009793]